{
  "gene_name": "Proteasome adapter and scaffold protein ECM29",
  "term_label": "ERAD pathway",
  "gene": "UniProtKB:Q5VYK3",
  "term_id": "GO:0036503",
  "gene_symbol": "ECPAS"
}